{
  "gene": "UniProtKB:Q9NQT5",
  "gene_symbol": "EXOSC3",
  "term_id": "GO:0000176",
  "gene_name": "Exosome complex component RRP40",
  "term_label": "nuclear exosome (RNase complex)"
}